{
  "term_label": "desmosome",
  "gene_name": "Desmocollin-2",
  "gene_symbol": "DSC2",
  "gene": "UniProtKB:Q02487",
  "term_id": "GO:0030057"
}